{
  "gene_name": "SH3 domain-binding protein 5-like",
  "term_label": "cytoplasm",
  "gene": "UniProtKB:Q7L8J4",
  "term_id": "GO:0005737",
  "gene_symbol": "SH3BP5L"
}